{
  "term_label": "positive regulation of synapse assembly",
  "term_id": "GO:0051965",
  "gene_name": "Reticulon-4 receptor-like 1",
  "gene_symbol": "RTN4RL1",
  "gene": "UniProtKB:Q86UN2"
}